glycosylceramide metabolic process [GO:0006677] (biological process) Also known as: glycosylceramide metabolism Definition: The chemical reactions and pathways involving glycosylceramides, any compound formed by the replacement of the glycosidic hydroxyl group of a cyclic form of a monosaccharide (or derivative) by a ceramide group. Relationships: is a type of ceramide metabolic process [GO:0006672]; is_a glycosphingolipid metabolic process [GO:0006687] Subtypes: glucosylceramide metabolic process [GO:0006678], galactosylceramide metabolic process [GO:0006681], glycosylceramide catabolic process [GO:0046477] Sources: GOC:ai, ISBN:0198506732